{
  "gene": "UniProtKB:Q9UN79",
  "gene_name": "Transcription factor SOX-13",
  "term_label": "cell fate commitment",
  "term_id": "GO:0045165",
  "gene_symbol": "SOX13"
}